esophagus development [GO:1903702] (biological process) Relationships: is a type of anatomical structure development [GO:0048856] Sources: GOC:TermGenie, GO_REF:0000094, ISBN:0-683-40008-8 Definition: The process whose specific outcome is the progression of an esophagus over time, from its formation to the mature structure. Also known as: esophageal development, gullet development, oesophagus development